{
  "gene_symbol": "LEF1",
  "term_label": "canonical Wnt signaling pathway",
  "gene": "UniProtKB:Q9UJU2",
  "gene_name": "Lymphoid enhancer-binding factor 1",
  "term_id": "GO:0060070"
}